{
  "gene": "UniProtKB:Q9UPQ7",
  "gene_name": "E3 ubiquitin-protein ligase PDZRN3",
  "term_id": "GO:0061630",
  "term_label": "ubiquitin protein ligase activity",
  "gene_symbol": "PDZRN3"
}